{
  "gene_symbol": "KLHL32",
  "term_id": "GO:1990756",
  "gene_name": "Kelch-like protein 32",
  "term_label": "ubiquitin-like ligase-substrate adaptor activity",
  "gene": "UniProtKB:Q96NJ5"
}